nucleoside phosphoacylhydrolase activity [GO:0033974] (molecular function) Relationships: is a type of hydrolase activity, acting on acid anhydrides, in phosphorus-containing anhydrides [GO:0016818] Definition: Catalysis of the hydrolysis of mixed phospho-anhydride bonds. Also known as: nucleoside-5'-phosphoacylate acylhydrolase activity Sources: EC:3.6.1.24